{
  "gene": "UniProtKB:O95190",
  "term_label": "nucleus",
  "term_id": "GO:0005634",
  "gene_name": "Ornithine decarboxylase antizyme 2",
  "gene_symbol": "OAZ2"
}